{
  "gene_name": "Phospholipid phosphatase 4",
  "gene": "UniProtKB:Q5VZY2",
  "term_label": "membrane",
  "gene_symbol": "PLPP4",
  "term_id": "GO:0016020"
}